{
  "gene_symbol": "SEMA4A",
  "term_id": "GO:0071526",
  "gene": "UniProtKB:Q9H3S1",
  "term_label": "semaphorin-plexin signaling pathway",
  "gene_name": "Semaphorin-4A"
}